{
  "gene": "UniProtKB:Q9NY59",
  "gene_name": "Sphingomyelin phosphodiesterase 3",
  "term_id": "GO:0004767",
  "gene_symbol": "SMPD3",
  "term_label": "sphingomyelin phosphodiesterase activity"
}